{
  "gene_symbol": "CCS",
  "gene_name": "Copper chaperone for superoxide dismutase",
  "term_label": "superoxide dismutase copper chaperone activity",
  "term_id": "GO:0016532",
  "gene": "UniProtKB:O14618"
}